{
  "term_id": "GO:0035556",
  "term_label": "intracellular signal transduction",
  "gene_name": "Protein phosphatase inhibitor 2 family member C",
  "gene_symbol": "PPP1R2C",
  "gene": "UniProtKB:O14990"
}